{
  "gene_symbol": "IRS4",
  "gene": "UniProtKB:O14654",
  "gene_name": "Insulin receptor substrate 4",
  "term_label": "plasma membrane",
  "term_id": "GO:0005886"
}